{
  "term_label": "transcription corepressor activity",
  "term_id": "GO:0003714",
  "gene": "UniProtKB:Q96SI1",
  "gene_symbol": "KCTD15",
  "gene_name": "BTB_POZ domain-containing protein KCTD15"
}